protein tyrosine kinase activity [GO:0004713] (molecular function) Also known as: protein-tyrosine kinase activity Regulation: negatively regulated by protein tyrosine kinase inhibitor activity [GO:0030292]; positively regulated by GO:0030296; regulated by GO:0061097; positively regulated by positive regulation of protein tyrosine kinase activity [GO:0061098]; negatively regulated by GO:0061099 Definition: Catalysis of the reaction: ATP + a protein tyrosine = ADP + protein tyrosine phosphate. Subtypes: transmembrane receptor protein tyrosine kinase activity [GO:0004714], GO:0004715, histone H3Y41 kinase activity [GO:0035401], GO:0140801 Relationships: is a type of protein kinase activity [GO:0004672] Sources: RHEA:10596